L-methionine biosynthetic process from L-homoserine via cystathionine [GO:0019279] (biological process) Relationships: is a type of homoserine metabolic process [GO:0009092]; is a type of 'de novo' L-methionine biosynthetic process [GO:0071266]; is a type of non-proteinogenic amino acid metabolic process [GO:0170041] Also known as: L-methionine anabolism from L-homoserine via cystathionine, L-methionine formation from L-homoserine via cystathionine, L-methionine synthesis from L-homoserine via cystathionine, methionine biosynthetic process from L-homoserine via cystathionine Definition: The chemical reactions and pathways resulting in the formation of L-methionine from L-homoserine, via the intermediate cystathionine. Sources: GOC:go_curators, MetaCyc:HOMOSER-METSYN-PWY Subtypes: L-methionine biosynthetic process from homoserine via O-succinyl-L-homoserine and cystathionine [GO:0019281], GO:0033516